diacylglycerol lipase activity [GO:0120516] (molecular function) Sources: RHEA:32731 Definition: Catalysis of the reaction: a diacylglycerol + H2O = a fatty acid + a monoacylglycerol + H+. Relationships: is a type of lipase activity [GO:0016298]